{
  "gene_symbol": "RUNDC1",
  "gene_name": "RUN domain-containing protein 1",
  "gene": "UniProtKB:Q96C34",
  "term_label": "Unknown cellular component",
  "term_id": "UNKNOWN:0003"
}